{
  "term_label": "epithelial cell differentiation",
  "term_id": "GO:0030855",
  "gene": "UniProtKB:P19012",
  "gene_name": "Keratin, type I cytoskeletal 15",
  "gene_symbol": "KRT15"
}